prepupal development [GO:0035210] (biological process) Definition: The process whose specific outcome is the progression of the prepupa over time, from its formation to the mature structure. The prepupal stage is a life stage interposed between the larval and the pupal stages in insects that undergo a complete metamorphosis. The start of the pre-pupal stage is marked by pupariation, and the end is marked by pupation. Sources: GOC:mtg_sensu, http://sdb.bio.purdue.edu/fly/aimain/1adult.htm Note: See also the fly_anatomy.ontology term 'prepupa ; FBbt:00002952'. Relationships: is a type of instar larval or pupal development [GO:0002165]